{
  "term_id": "GO:0016020",
  "gene": "UniProtKB:Q96J65",
  "gene_symbol": "ABCC12",
  "term_label": "membrane",
  "gene_name": "ATP-binding cassette sub-family C member 12"
}